negative regulation of organ growth [GO:0046621] (biological process) Relationships: is_a regulation of organ growth [GO:0046620]; is a type of GO:0048640; is a type of negative regulation of multicellular organismal process [GO:0051241]; negatively regulates organ growth [GO:0035265] Subtypes: negative regulation of heart growth [GO:0061117], GO:0061914 Sources: GOC:bf, GOC:tb Definition: Any process that stops, prevents, or reduces the frequency, rate or extent of growth of an organ of an organism.